{
  "gene_symbol": "TIMM23B",
  "gene": "UniProtKB:Q5SRD1",
  "term_id": "GO:0008320",
  "term_label": "protein transmembrane transporter activity",
  "gene_name": "Mitochondrial import inner membrane translocase subunit Tim23B"
}